{
  "gene": "UniProtKB:Q7RTU3",
  "term_id": "GO:0061564",
  "gene_symbol": "OLIG3",
  "term_label": "axon development",
  "gene_name": "Oligodendrocyte transcription factor 3"
}